negative regulation of chronic inflammatory response [GO:0002677] (biological process) Relationships: is a type of GO:0002676; is a type of GO:0050728; negatively regulates chronic inflammatory response [GO:0002544] Sources: GOC:add Also known as: down regulation of chronic inflammatory response, down-regulation of chronic inflammatory response, downregulation of chronic inflammatory response, inhibition of chronic inflammatory response Subtypes: negative regulation of granuloma formation [GO:0002632], GO:0002875, negative regulation of chronic inflammatory response to non-antigenic stimulus [GO:0002881] Definition: Any process that stops, prevents, or reduces the frequency, rate, or extent of a chronic inflammatory response.